{
  "gene_name": "Myosin-binding protein C, cardiac-type",
  "term_id": "GO:0045214",
  "term_label": "sarcomere organization",
  "gene_symbol": "MYBPC3",
  "gene": "UniProtKB:Q14896"
}